{
  "gene_name": "Large ribosomal subunit protein uL14m",
  "gene_symbol": "MRPL14",
  "gene": "UniProtKB:Q6P1L8",
  "term_id": "UNKNOWN:0001",
  "term_label": "Unknown molecular function"
}